{
  "gene_symbol": "PCDHGC4",
  "term_id": "GO:0050839",
  "gene": "UniProtKB:Q9Y5F7",
  "gene_name": "Protocadherin gamma-C4",
  "term_label": "cell adhesion molecule binding"
}